{
  "gene": "UniProtKB:O43752",
  "term_label": "retrograde transport, endosome to Golgi",
  "term_id": "GO:0042147",
  "gene_symbol": "STX6",
  "gene_name": "Syntaxin-6"
}